{
  "term_label": "cytoplasm",
  "term_id": "GO:0005737",
  "gene": "UniProtKB:Q9BXL6",
  "gene_name": "Caspase recruitment domain-containing protein 14",
  "gene_symbol": "CARD14"
}